{
  "gene_symbol": "TMF1",
  "gene": "UniProtKB:P82094",
  "term_label": "Golgi apparatus",
  "gene_name": "TATA element modulatory factor",
  "term_id": "GO:0005794"
}